phosphorus metabolic process [GO:0006793] (biological process) Regulation: positively regulated by GO:0010562; negatively regulated by negative regulation of phosphorus metabolic process [GO:0010563]; regulated by GO:0051174 Definition: The chemical reactions and pathways involving the nonmetallic element phosphorus or compounds that contain phosphorus. Subtypes: phosphorus utilization [GO:0006794], GO:0006796, GO:0006797, glyphosate metabolic process [GO:0018920], GO:0019298, GO:0019634, 2-aminoethylphosphonate catabolic process [GO:0019635], phosphonoacetate metabolic process [GO:0019636], GO:0019637, diphosphate metabolic process [GO:0071344], tatiopterin metabolic process [GO:1900869], sulfurated eukaryotic molybdenum cofactor(2-) biosynthetic process [GO:1902756] Relationships: is a type of metabolic process [GO:0008152] Also known as: phosphorus metabolism Sources: GOC:ai